{
  "gene_symbol": "AGA",
  "term_label": "lysosome",
  "term_id": "GO:0005764",
  "gene": "UniProtKB:P20933",
  "gene_name": "N(4)-(beta-N-acetylglucosaminyl)-L-asparaginase"
}